{
  "gene_name": "Myb_SANT-like DNA-binding domain-containing protein 2",
  "term_label": "Unknown cellular component",
  "gene": "UniProtKB:Q6P1R3",
  "term_id": "UNKNOWN:0003",
  "gene_symbol": "MSANTD2"
}